positive regulation of extrinsic apoptotic signaling pathway [GO:2001238] (biological process) Definition: Any process that activates or increases the frequency, rate or extent of extrinsic apoptotic signaling pathway. Relationships: is a type of positive regulation of apoptotic signaling pathway [GO:2001235]; is a type of regulation of extrinsic apoptotic signaling pathway [GO:2001236]; positively regulates GO:0097191 Also known as: positive regulation of extrinsic apoptotic signalling pathway, positive regulation of extrinsic apoptosis Sources: GOC:mtg_apoptosis Subtypes: positive regulation of extrinsic apoptotic signaling pathway via death domain receptors [GO:1902043], positive regulation of extrinsic apoptotic signaling pathway in absence of ligand [GO:2001241]